{
  "gene_symbol": "MTMR6",
  "gene": "UniProtKB:Q9Y217",
  "gene_name": "Myotubularin-related protein 6",
  "term_label": "nuclear envelope",
  "term_id": "GO:0005635"
}